acetate-CoA ligase activity [GO:0003987] (molecular function) Relationships: is a type of CoA-ligase activity [GO:0016405]; is a type of GO:0016878 Sources: EC:6.2.1.1 Definition: Catalysis of the reaction: ATP + acetate + CoA = AMP + diphosphate + acetyl-CoA. Also known as: acetate thiokinase activity, acyl-activating enzyme activity, ACS, acetate to acetyl-CoA, acetate:CoA ligase (AMP-forming), acetic thiokinase activity, acetyl CoA ligase activity, acetyl CoA synthase activity, acetyl activating enzyme, acetyl coenzyme A synthetase activity, acetyl-CoA synthase activity, acetyl-CoA synthetase activity, acetyl-activating enzyme activity, acetyl-coenzyme A synthase activity, short chain fatty acyl-CoA synthetase activity, short-chain acyl-coenzyme A synthetase activity